{
  "term_id": "GO:0000981",
  "gene_name": "T-box transcription factor TBX4",
  "gene": "UniProtKB:P57082",
  "gene_symbol": "TBX4",
  "term_label": "DNA-binding transcription factor activity, RNA polymerase II-specific"
}